{
  "gene_symbol": "UBAP2L",
  "gene_name": "Ubiquitin-associated protein 2-like",
  "gene": "UniProtKB:Q14157",
  "term_id": "UNKNOWN:0001",
  "term_label": "Unknown molecular function"
}